{
  "term_id": "GO:0031663",
  "gene_symbol": "IRAK1",
  "gene_name": "Interleukin-1 receptor-associated kinase 1",
  "term_label": "lipopolysaccharide-mediated signaling pathway",
  "gene": "UniProtKB:P51617"
}